{
  "term_label": "glutamatergic synapse",
  "term_id": "GO:0098978",
  "gene_name": "Adhesion G protein-coupled receptor A1",
  "gene_symbol": "ADGRA1",
  "gene": "UniProtKB:Q86SQ6"
}